{
  "gene": "UniProtKB:Q7Z6E9",
  "term_id": "GO:0061630",
  "term_label": "ubiquitin protein ligase activity",
  "gene_symbol": "RBBP6",
  "gene_name": "E3 ubiquitin-protein ligase RBBP6"
}